{
  "gene_name": "F-box only protein 44",
  "term_id": "GO:0036503",
  "gene_symbol": "FBXO44",
  "gene": "UniProtKB:Q9H4M3",
  "term_label": "ERAD pathway"
}